{
  "gene_symbol": "IKBKG",
  "gene": "UniProtKB:Q9Y6K9",
  "term_label": "cytoplasm",
  "gene_name": "NF-kappa-B essential modulator",
  "term_id": "GO:0005737"
}